GDP-dissociation inhibitor activity [GO:0005092] (MF) Also known as: GDI Relationships: is a type of GTPase regulator activity [GO:0030695]; positively regulates GDP binding [GO:0019003] Definition: Prevents the dissociation of GDP from a GTPase, thereby preventing GTP from binding. Sources: GOC:mah Subtypes: GO:0005093, GO:0005094